{
  "term_label": "antigen processing and presentation of exogenous peptide antigen via MHC class I",
  "gene": "UniProtKB:P30273",
  "gene_symbol": "FCER1G",
  "term_id": "GO:0042590",
  "gene_name": "High affinity immunoglobulin epsilon receptor subunit gamma"
}